{
  "term_label": "chromatin binding",
  "term_id": "GO:0003682",
  "gene_symbol": "BRD3",
  "gene_name": "Bromodomain-containing protein 3",
  "gene": "UniProtKB:Q15059"
}